{
  "term_label": "structural constituent of muscle",
  "term_id": "GO:0008307",
  "gene_symbol": "MYOM2",
  "gene": "UniProtKB:P54296",
  "gene_name": "Myomesin-2"
}